GID complex [GO:0034657] (CC) Relationships: is a type of ubiquitin ligase complex [GO:0000151] Also known as: C-terminal to LisH complex, CTLH complex References: PMID:12686616, PMID:18508925, PMID:35682545 Definition: A protein complex with ubiquitin ligase activity that, in Saccharomyces cerevisiae, is involved in proteasomal degradation of fructose-1,6-bisphosphatase (FBPase) and phosphoenolpyruvate carboxykinase during the transition from gluconeogenic to glycolytic growth conditions. It appears to play a broader role in cellular homeostasis and development in other species.